regulation of DNA amplification [GO:1904523] (biological process) Relationships: is_a regulation of DNA biosynthetic process [GO:2000278]; regulates DNA amplification [GO:0006277] Subtypes: negative regulation of DNA amplification [GO:1904524], positive regulation of DNA amplification [GO:1904525] Definition: Any process that modulates the frequency, rate or extent of DNA amplification. References: PMID:26195783 Sources: GOC:TermGenie, GO_REF:0000058